{
  "gene": "UniProtKB:A0A087X179",
  "term_label": "Unknown cellular component",
  "gene_symbol": "TBC1D3E",
  "term_id": "UNKNOWN:0003",
  "gene_name": "TBC1 domain family member 3E"
}